{
  "term_id": "UNKNOWN:0003",
  "gene_symbol": "SPDYE15",
  "gene_name": "Putative speedy protein E15",
  "gene": "UniProtKB:P0DUD4",
  "term_label": "Unknown cellular component"
}